mammary gland duct cavitation [GO:0060604] (biological process) Relationships: is a type of tube lumen cavitation [GO:0060605]; is part of mammary gland duct morphogenesis [GO:0060603] Definition: Creation of the central hole of the mammary gland duct by the hollowing out of a solid rod. References: PMID:17120154 Sources: GOC:dph Also known as: milk duct cavitation